{
  "gene_symbol": "TBC1D20",
  "gene_name": "TBC1 domain family member 20",
  "term_label": "GTPase activator activity",
  "term_id": "GO:0005096",
  "gene": "UniProtKB:Q96BZ9"
}